{
  "term_id": "GO:0005737",
  "term_label": "cytoplasm",
  "gene_symbol": "NPPB",
  "gene": "UniProtKB:P16860",
  "gene_name": "Natriuretic peptides B"
}